abducens nerve maturation [GO:0021601] (biological process) Also known as: CN VI maturation Sources: GOC:cls, GOC:dgh, GOC:dph, GOC:jid, GO_REF:0000021 Relationships: is a type of GO:0021605; is part of abducens nerve development [GO:0021560] Definition: A developmental process, independent of morphogenetic (shape) change, that is required for the abducens nerve to attain its fully functional state. The motor function of the abducens nerve is to contract the lateral rectus which results in abduction of the eye.